FAD-dependent H3K4me/H3K4me3 demethylase activity [GO:0140682] (molecular function) Also known as: histone H3K4me2 demethylase activity, histone H3-di/monomethyl-lysine-4 FAD-dependent demethylase activity, histone H3K4me demethylase activity Definition: Catalysis of the removal of a methyl group from a di- or a monomethyl-lysine residue at position 4 of the histone H3 protein. This is a flavin adenine dinucleotide (FAD)-dependent amine oxidation reaction. Note: Comment: Note that the residue position corresponds to the canonical human H3 histone (UniProtKB:P84243); this residue is conserved across all eukaryotes. Residue 1 is the first residue following removal of the initiating Methionine (Met). Note that each histone is encoded by multiple genes, and sequences may vary across different genes within an organism. Relationships: is a type of oxidoreductase activity, acting on paired donors, with incorporation or reduction of molecular oxygen [GO:0016705]; is a type of GO:0032453 References: PMID:22473470